interleukin-8 production [GO:0032637] (biological process) Also known as: IL-8 production, interleukin-8 biosynthetic process, interleukin-8 secretion Sources: GOC:mah Definition: The appearance of interleukin-8 due to biosynthesis or secretion following a cellular stimulus, resulting in an increase in its intracellular or extracellular levels. Relationships: is a type of GO:0001816 Regulation: regulated by regulation of interleukin-8 production [GO:0032677]; negatively regulated by negative regulation of interleukin-8 production [GO:0032717]; positively regulated by positive regulation of interleukin-8 production [GO:0032757]